{
  "term_id": "GO:0000981",
  "gene_name": "Zinc finger protein 546",
  "gene": "UniProtKB:Q86UE3",
  "term_label": "DNA-binding transcription factor activity, RNA polymerase II-specific",
  "gene_symbol": "ZNF546"
}